anaerobic respiration [GO:0009061] (biological process) Subtypes: methanogenesis [GO:0015948], anaerobic respiration, using ammonium as electron donor [GO:0019331], dissimilatory sulfate reduction [GO:0019420] Definition: The enzymatic release of energy from inorganic and organic compounds (especially carbohydrates and fats) which uses compounds other than oxygen (e.g. nitrate, sulfate) as the terminal electron acceptor. Relationships: is a type of cellular respiration [GO:0045333] Sources: GOC:das, GOC:jl, ISBN:0140513590